regulation of angiogenesis [GO:0045765] (biological process) Definition: Any process that modulates the frequency, rate or extent of angiogenesis. Sources: GOC:go_curators Subtypes: negative regulation of angiogenesis [GO:0016525], GO:0045766, regulation of vascular wound healing [GO:0061043], regulation of sprouting angiogenesis [GO:1903670], regulation of blood vessel branching [GO:1905553] Relationships: is a type of regulation of anatomical structure morphogenesis [GO:0022603]; is a type of regulation of vasculature development [GO:1901342]; regulates angiogenesis [GO:0001525]